{
  "term_id": "GO:0006672",
  "gene_symbol": "CERK",
  "term_label": "ceramide metabolic process",
  "gene_name": "Ceramide kinase",
  "gene": "UniProtKB:Q8TCT0"
}